{
  "gene_symbol": "OVOS1",
  "gene": "UniProtKB:Q6IE37",
  "gene_name": "Ovostatin homolog 1",
  "term_label": "Unknown molecular function",
  "term_id": "UNKNOWN:0001"
}